{
  "term_id": "GO:0019903",
  "gene_symbol": "JUP",
  "gene": "UniProtKB:P14923",
  "term_label": "protein phosphatase binding",
  "gene_name": "Junction plakoglobin"
}